{
  "gene_name": "Tetratricopeptide repeat protein 17",
  "term_id": "UNKNOWN:0001",
  "term_label": "Unknown molecular function",
  "gene_symbol": "TTC17",
  "gene": "UniProtKB:Q96AE7"
}